negative regulation of blood vessel remodeling [GO:0060313] (biological process) Also known as: down-regulation of blood vessel remodeling, negative regulation of blood vessel remodelling, inhibition of blood vessel remodeling Relationships: is a type of negative regulation of tissue remodeling [GO:0034104]; is a type of negative regulation of developmental process [GO:0051093]; is a type of GO:0060312; negatively regulates GO:0001974 Subtypes: negative regulation of pulmonary blood vessel remodeling [GO:1905110] Sources: GOC:BHF, GOC:dph, GOC:tb Definition: Any process that decreases the rate, frequency or extent of blood vessel remodeling, the reorganization or renovation of existing blood vessels.